{
  "gene": "UniProtKB:Q8NBL3",
  "gene_name": "Transmembrane protein 178A",
  "gene_symbol": "TMEM178A",
  "term_id": "GO:0045671",
  "term_label": "negative regulation of osteoclast differentiation"
}